{
  "gene_name": "Testis-specific chromodomain protein Y 1",
  "gene_symbol": "CDY1B",
  "term_id": "GO:0062072",
  "term_label": "histone H3K9me2/3 reader activity",
  "gene": "UniProtKB:Q9Y6F8"
}